{
  "term_id": "GO:0005759",
  "gene_symbol": "ACSM5",
  "term_label": "mitochondrial matrix",
  "gene_name": "Acyl-coenzyme A synthetase ACSM5, mitochondrial",
  "gene": "UniProtKB:Q6NUN0"
}